{
  "gene": "UniProtKB:Q5TCS8",
  "term_id": "GO:0006225",
  "term_label": "UDP biosynthetic process",
  "gene_name": "Adenylate kinase 9",
  "gene_symbol": "AK9"
}